{
  "gene_name": "Tumor protein 63",
  "gene": "UniProtKB:Q9H3D4",
  "term_label": "positive regulation of transcription by RNA polymerase II",
  "term_id": "GO:0045944",
  "gene_symbol": "TP63"
}